{
  "gene": "UniProtKB:Q6ZSR3",
  "gene_name": "Putative uncharacterized protein FLJ45275, mitochondrial",
  "term_label": "Unknown cellular component",
  "gene_symbol": "Q6ZSR3",
  "term_id": "UNKNOWN:0003"
}